{
  "gene_name": "Stromal membrane-associated protein 2",
  "term_id": "UNKNOWN:0002",
  "gene": "UniProtKB:Q8WU79",
  "term_label": "Unknown biological process",
  "gene_symbol": "SMAP2"
}